{
  "gene_name": "DNA helicase B",
  "gene_symbol": "HELB",
  "term_label": "Unknown cellular component",
  "gene": "UniProtKB:Q8NG08",
  "term_id": "UNKNOWN:0003"
}